{
  "gene": "UniProtKB:Q96MY7",
  "gene_symbol": "FAM161B",
  "term_label": "cilium organization",
  "term_id": "GO:0044782",
  "gene_name": "Protein FAM161B"
}